{
  "gene_name": "Receptor expression-enhancing protein 4",
  "gene_symbol": "REEP4",
  "term_id": "GO:0005789",
  "term_label": "endoplasmic reticulum membrane",
  "gene": "UniProtKB:Q9H6H4"
}